{
  "term_id": "UNKNOWN:0001",
  "gene_name": "Immunoglobulin lambda variable 5-37",
  "term_label": "Unknown molecular function",
  "gene_symbol": "IGLV5-37",
  "gene": "UniProtKB:A0A075B6J1"
}